{
  "gene": "UniProtKB:O00478",
  "term_label": "signaling receptor binding",
  "gene_symbol": "BTN3A3",
  "term_id": "GO:0005102",
  "gene_name": "Butyrophilin subfamily 3 member A3"
}